{
  "gene_symbol": "C3orf33",
  "term_label": "extracellular space",
  "gene": "UniProtKB:Q6P1S2",
  "gene_name": "Protein C3orf33",
  "term_id": "GO:0005615"
}